phospholipase C-activating G protein-coupled glutamate receptor signaling pathway [GO:0007206] (biological process) Also known as: activation of phospholipase C activity by G-protein coupled glutamate receptor signaling pathway, activation of phospholipase C activity by metabotropic glutamate receptor signaling pathway, activation of phospholipase C activity by metabotropic glutamate receptor signalling pathway, metabotropic glutamate receptor, phospholipase C activating pathway, phospholipase C-activating G-protein coupled glutamate receptor signaling pathway Relationships: is a type of GO:0007200; is a type of GO:0007216; has part PLC activating G protein-coupled glutamate receptor activity [GO:0001639] Definition: A phospholipase C-activating G protein-coupled receptor signaling pathway initiated by glutamate binding to its receptor on the surface of a target cell, and ending with the regulation of a downstream cellular process, e.g. transcription. Sources: GOC:dph, GOC:mah, GOC:signaling, GOC:tb